{
  "gene": "UniProtKB:Q1A5X6",
  "gene_symbol": "IQCJ",
  "term_label": "Unknown cellular component",
  "gene_name": "IQ domain-containing protein J",
  "term_id": "UNKNOWN:0003"
}